{
  "term_label": "Unknown biological process",
  "term_id": "UNKNOWN:0002",
  "gene": "UniProtKB:P35475",
  "gene_name": "Alpha-L-iduronidase",
  "gene_symbol": "IDUA"
}